Lewis a epitope biosynthetic process [GO:0010493] (biological process) Relationships: is a type of polysaccharide biosynthetic process [GO:0000271]; is a type of carbohydrate derivative biosynthetic process [GO:1901137] Definition: The chemical reactions and pathways resulting in the formation of a Lewis a epitope, a trisaccharide (Fuc-alpha-(1->4)[Gal-beta-(1->3)]GlcNAc) characteristic of plant protein N-linked oligosaccharides. Also known as: LE A biosynthetic process References: PMID:17630273